host cell lysosomal membrane [GO:0044188] (cellular component) Definition: The lipid bilayer surrounding the host cell lysosome and separating its contents from the host cell cytoplasm. Relationships: is_a host cell membrane [GO:0033644]; is part of host cell lysosome [GO:0044187] Sources: GOC:jl